{
  "gene_name": "Protein kinase C alpha type",
  "term_label": "Unknown cellular component",
  "gene": "UniProtKB:P17252",
  "term_id": "UNKNOWN:0003",
  "gene_symbol": "PRKCA"
}